{
  "gene_symbol": "NBPF3",
  "term_id": "UNKNOWN:0003",
  "term_label": "Unknown cellular component",
  "gene_name": "Neuroblastoma breakpoint family member 3",
  "gene": "UniProtKB:Q9H094"
}